{
  "gene": "UniProtKB:O75467",
  "term_id": "GO:0006357",
  "gene_name": "Zinc finger protein 324A",
  "gene_symbol": "ZNF324",
  "term_label": "regulation of transcription by RNA polymerase II"
}